{
  "gene_name": "Scavenger receptor class A member 5",
  "gene_symbol": "SCARA5",
  "term_label": "ferritin receptor activity",
  "gene": "UniProtKB:Q6ZMJ2",
  "term_id": "GO:0070287"
}